{
  "term_id": "GO:0005654",
  "term_label": "nucleoplasm",
  "gene_symbol": "ZBTB17",
  "gene_name": "Zinc finger and BTB domain-containing protein 17",
  "gene": "UniProtKB:Q13105"
}